positive regulation of retinal ganglion cell axon guidance [GO:1902336] (biological process) Also known as: positive regulation of retinal ganglion cell axon pathfinding, up regulation of retinal ganglion cell axon guidance, up regulation of retinal ganglion cell axon pathfinding, up-regulation of retinal ganglion cell axon guidance, up-regulation of retinal ganglion cell axon pathfinding, upregulation of retinal ganglion cell axon guidance, upregulation of retinal ganglion cell axon pathfinding, activation of retinal ganglion cell axon guidance, activation of retinal ganglion cell axon pathfinding Definition: Any process that activates or increases the frequency, rate or extent of retinal ganglion cell axon guidance. References: PMID:21658587 Sources: GOC:BHF, GOC:TermGenie, GOC:rl Relationships: is a type of regulation of retinal ganglion cell axon guidance [GO:0090259]; is a type of positive regulation of axon guidance [GO:1902669]; positively regulates retinal ganglion cell axon guidance [GO:0031290]